{
  "gene_name": "Microspherule protein 1",
  "term_id": "GO:0044545",
  "term_label": "NSL complex",
  "gene_symbol": "MCRS1",
  "gene": "UniProtKB:Q96EZ8"
}